{
  "gene": "UniProtKB:P31327",
  "gene_symbol": "CPS1",
  "term_label": "carbamoyl-phosphate synthase (ammonia) activity",
  "gene_name": "Carbamoyl-phosphate synthase [ammonia], mitochondrial",
  "term_id": "GO:0004087"
}